glutamine N-acyltransferase activity [GO:0047946] (molecular function) Sources: EC:2.3.1.68, MetaCyc:GLUTAMINE-N-ACYLTRANSFERASE-RXN Also known as: acyl-CoA:L-glutamine N-acyltransferase activity Definition: Catalysis of the reaction: acyl-CoA + L-glutamine = CoA + N-acyl-L-glutamine. Relationships: is a type of N-acyltransferase activity [GO:0016410]